alizarin 2-beta-glucosyltransferase activity [GO:0047644] (molecular function) Also known as: alizarin 2-b-glucosyltransferase activity, UDP-glucose:1,2-dihydroxy-9,10-anthraquinone 2-O-beta-D-glucosyltransferase activity, UDPglucose:1,2-dihydroxy-9,10-anthraquinone 2-O-beta-D-glucosyl-transferase activity, uridine diphosphoglucose-alizarin glucosyltransferase activity Definition: Catalysis of the reaction: alizarin + UDP-D-glucose = 1-hydroxy-2-(beta-D-glucosyloxy)-9,10-anthraquinone + H+ + UDP. Sources: EC:2.4.1.103, RHEA:20677 Relationships: is a type of GO:0035251